{
  "term_label": "DNA-binding transcription factor activity, RNA polymerase II-specific",
  "term_id": "GO:0000981",
  "gene_name": "Hepatocyte nuclear factor 3-gamma",
  "gene_symbol": "FOXA3",
  "gene": "UniProtKB:P55318"
}